{
  "gene": "UniProtKB:Q9H0W9",
  "term_id": "GO:0005634",
  "gene_name": "Ester hydrolase C11orf54",
  "term_label": "nucleus",
  "gene_symbol": "C11orf54"
}